mRNA splicing, via endonucleolytic cleavage and ligation [GO:0070054] (biological process) Also known as: cytosolic mRNA splicing Relationships: is a type of RNA splicing, via endonucleolytic cleavage and ligation [GO:0000394]; is a type of GO:0006397 Note: Note that while typically associated with tRNA splicing, splicing via endonucleolytic cleavages and subsequent ligation of the free exon ends is known to be used for some non-tRNA substrates, e.g. HAC1 (YFL031W) in S. cerevisiae and an intron in the 23S rRNA of the Archaeal species Desulfurococcus mobilis. Sources: GOC:krc, GOC:mah Definition: Splicing of mRNA substrates via recognition of the folded RNA structure that brings the 5' and 3' splice sites into proximity and cleavage of the RNA at both the 3' and 5' splice sites by an endonucleolytic mechanism, followed by ligation of the exons.